{
  "gene_name": "Myb-related transcription factor, partner of profilin",
  "gene": "UniProtKB:Q86VE0",
  "gene_symbol": "MYPOP",
  "term_label": "nucleus",
  "term_id": "GO:0005634"
}